camalexin binding [GO:2001147] (molecular function) Definition: Binding to camalexin. Sources: GOC:obol Also known as: 3-(1,3-thiazol-2-yl)-1H-indole binding Relationships: is a type of sulfur compound binding [GO:1901681]